{
  "gene_symbol": "SIX4",
  "gene_name": "Homeobox protein SIX4",
  "term_id": "GO:0005667",
  "term_label": "transcription regulator complex",
  "gene": "UniProtKB:Q9UIU6"
}